{
  "gene_symbol": "P2RY4",
  "term_label": "plasma membrane",
  "gene_name": "P2Y purinoceptor 4",
  "gene": "UniProtKB:P51582",
  "term_id": "GO:0005886"
}